{
  "gene_symbol": "ZPR1",
  "gene_name": "Zinc finger protein ZPR1",
  "term_label": "cytoplasm",
  "gene": "UniProtKB:O75312",
  "term_id": "GO:0005737"
}